{
  "term_id": "GO:0071004",
  "gene": "UniProtKB:A8MWD9",
  "gene_name": "Putative small nuclear ribonucleoprotein G-like protein 15",
  "gene_symbol": "SNRPGP15",
  "term_label": "U2-type prespliceosome"
}